{
  "gene_name": "Cyclic nucleotide-gated cation channel alpha-4",
  "gene_symbol": "CNGA4",
  "term_id": "GO:0007606",
  "gene": "UniProtKB:Q8IV77",
  "term_label": "sensory perception of chemical stimulus"
}